{
  "gene_symbol": "CDS1",
  "term_id": "GO:0140042",
  "term_label": "lipid droplet formation",
  "gene_name": "Phosphatidate cytidylyltransferase 1",
  "gene": "UniProtKB:Q92903"
}